label approved by the SynGO project [go#syngo:official:label]